norepinephrine transport [GO:0015874] (biological process) Also known as: levarterenol transport, noradrenaline transport Subtypes: norepinephrine secretion [GO:0048243], norepinephrine uptake [GO:0051620] Definition: The directed movement of norepinephrine into, out of or within a cell, or between cells, by means of some agent such as a transporter or pore. Norepinephrine (3,4-dihydroxyphenyl-2-aminoethanol) is a hormone secreted by the adrenal medulla and a neurotransmitter in the sympathetic peripheral nervous system and in some tracts of the CNS. It is also the biosynthetic precursor of epinephrine. Sources: GOC:ai, ISBN:0198506732 Relationships: is_a organic cation transport [GO:0015695]; is a type of GO:0051937